tRNA-uridine 2-sulfurtransferase activity [GO:0103016] (molecular function) Definition: Catalysis of the reaction: AH2 + ATP + S-sulfanyl-L-cysteinyl-[protein] + uridine(34) in tRNA = 2-thiouridine(34) in tRNA + A + AMP + diphosphate + H+ + L-cysteinyl-[protein]. Relationships: is a type of GO:0016783; is a type of catalytic activity, acting on a tRNA [GO:0140101] Also known as: tRNA-specific 2-thiouridylase activity, tRNA-uracil-34 sulfurtransferase activity Sources: RHEA:47032